positive regulation of purine nucleoside transport [GO:0032248] (biological process) Relationships: is a type of GO:0032244; is a type of regulation of purine nucleoside transport [GO:0032245] Definition: Any process that activates or increases the frequency, rate or extent of the directed movement of a purine nucleoside into, out of or within a cell, or between cells, by means of some agent such as a transporter or pore. Subtypes: positive regulation of adenosine transport [GO:0032251], positive regulation of inosine transport [GO:0035342] Sources: GOC:mah Also known as: up regulation of purine nucleoside transport, up-regulation of purine nucleoside transport, upregulation of purine nucleoside transport, activation of purine nucleoside transport, stimulation of purine nucleoside transport